{
  "gene": "UniProtKB:Q96QB1",
  "term_label": "actin cytoskeleton organization",
  "gene_name": "Rho GTPase-activating protein 7",
  "term_id": "GO:0030036",
  "gene_symbol": "DLC1"
}